{
  "gene_name": "WD repeat-containing protein 13",
  "term_label": "Unknown molecular function",
  "gene_symbol": "WDR13",
  "gene": "UniProtKB:Q9H1Z4",
  "term_id": "UNKNOWN:0001"
}